{
  "gene": "UniProtKB:Q9Y2G8",
  "term_id": "UNKNOWN:0003",
  "gene_symbol": "DNAJC16",
  "gene_name": "DnaJ homolog subfamily C member 16",
  "term_label": "Unknown cellular component"
}